{
  "gene_name": "Protein phosphatase 1 regulatory subunit 35",
  "gene": "UniProtKB:Q8TAP8",
  "term_label": "positive regulation of centriole elongation",
  "term_id": "GO:1903724",
  "gene_symbol": "PPP1R35"
}